negative regulation of plasminogen activation [GO:0010757] (biological process) Sources: GOC:BHF, GOC:dph, GOC:tb Relationships: is a type of regulation of plasminogen activation [GO:0010755]; is a type of GO:0010955; negatively regulates plasminogen activation [GO:0031639] Definition: Any process that decreases the rate, frequency or extent of plasminogen activation. Plasminogen activation is the process in which plasminogen is processed to plasmin. Also known as: inhibition of plasminogen activation